{
  "gene_name": "Leukocyte immunoglobulin-like receptor subfamily B member 4",
  "gene_symbol": "LILRB4",
  "term_label": "plasma membrane",
  "gene": "UniProtKB:Q8NHJ6",
  "term_id": "GO:0005886"
}